ABC-type oligogalacturonide transporter activity [GO:0033154] (molecular function) Definition: Enables the transfer of a solute or solutes from one side of a membrane to the other according to the reaction: ATP + H2O + oligogalacturonide(out) = ADP + phosphate + oligogalacturonide(in). References: PMID:11555291, PMID:17451747 Sources: GOC:mlg Also known as: oligogalacturonide-transporting ATPase activity, oligogalacturonide transmembrane transporter activity, ATP-dependent oligogalacturonide transmembrane transporter activity, ATPase-coupled oligogalacturonide transmembrane transporter activity, oligogalacturonide transporting ATPase activity Relationships: is_a ABC-type oligosaccharide transporter activity [GO:0015422]; is part of oligogalacturonide transport [GO:0033156]